{
  "gene_name": "Immunoglobulin heavy variable 1-8",
  "gene": "UniProtKB:P0DP01",
  "term_label": "Unknown cellular component",
  "gene_symbol": "IGHV1-8",
  "term_id": "UNKNOWN:0003"
}